{
  "term_id": "GO:0005886",
  "gene_name": "Germ cell-specific gene 1 protein",
  "term_label": "plasma membrane",
  "gene_symbol": "GSG1",
  "gene": "UniProtKB:Q2KHT4"
}